regulation of collateral sprouting [GO:0048670] (biological process) Subtypes: negative regulation of collateral sprouting [GO:0048671], positive regulation of collateral sprouting [GO:0048672], regulation of collateral sprouting of intact axon in response to injury [GO:0048683], GO:0048693, regulation of collateral sprouting in absence of injury [GO:0048696] Definition: Any process that modulates the frequency, rate or extent of collateral sprouting. Sources: GOC:dgh, GOC:dph, GOC:jid, GOC:lm Relationships: is_a regulation of developmental growth [GO:0048638]; is a type of regulation of axonogenesis [GO:0050770]; is a type of regulation of extent of cell growth [GO:0061387]; regulates collateral sprouting [GO:0048668]